{
  "gene_name": "Phospholipase A and acyltransferase 3",
  "gene": "UniProtKB:P53816",
  "term_label": "cytoplasm",
  "gene_symbol": "PLAAT3",
  "term_id": "GO:0005737"
}